{
  "gene_symbol": "ARRDC3",
  "gene_name": "Arrestin domain-containing protein 3",
  "term_label": "plasma membrane",
  "term_id": "GO:0005886",
  "gene": "UniProtKB:Q96B67"
}